tRNA export from nucleus [GO:0006409] (biological process) Subtypes: tRNA re-export from nucleus [GO:0071528] Relationships: is a type of RNA export from nucleus [GO:0006405]; is a type of tRNA transport [GO:0051031] Also known as: tRNA export from cell nucleus, tRNA export out of nucleus, tRNA transport from nucleus to cytoplasm, tRNA-nucleus export Definition: The directed movement of tRNA from the nucleus to the cytoplasm. Sources: GOC:ma Regulation: regulated by GO:2000238; negatively regulated by negative regulation of tRNA export from nucleus [GO:2000239]; positively regulated by positive regulation of tRNA export from nucleus [GO:2000240]